{
  "term_id": "GO:0001916",
  "gene_name": "Antigen-presenting glycoprotein CD1d",
  "term_label": "positive regulation of T cell mediated cytotoxicity",
  "gene": "UniProtKB:P15813",
  "gene_symbol": "CD1D"
}